{
  "term_label": "nuclear-transcribed mRNA catabolic process, nonsense-mediated decay",
  "gene_name": "Regulator of nonsense transcripts 2",
  "gene_symbol": "UPF2",
  "gene": "UniProtKB:Q9HAU5",
  "term_id": "GO:0000184"
}